homocysteine biosynthetic process [GO:0071268] (biological process) Also known as: homocysteine anabolism, homocysteine biosynthesis, homocysteine formation, homocysteine synthesis Subtypes: L-homocysteine biosynthetic process [GO:0071269] Definition: The chemical reactions and pathways resulting in the formation of homocysteine, 2-amino-4-sulfanylbutanoic acid. Sources: GOC:ecd, GOC:mah Relationships: is a type of sulfur amino acid biosynthetic process [GO:0000097]; is a type of homocysteine metabolic process [GO:0050667]; is_a non-proteinogenic amino acid biosynthetic process [GO:0170043]; is a type of GO:1901607